{
  "term_id": "GO:0003723",
  "gene": "UniProtKB:Q2NL82",
  "gene_name": "Pre-rRNA-processing protein TSR1 homolog",
  "gene_symbol": "TSR1",
  "term_label": "RNA binding"
}